17-O-deacetylvindoline O-acetyltransferase activity [GO:0047162] (molecular function) Relationships: is a type of O-acetyltransferase activity [GO:0016413] Sources: EC:2.3.1.107, RHEA:24496 Definition: Catalysis of the reaction: (1R,9R,10S,11R,12R,19R)-12-ethyl-10,11-dihydroxy-5-methoxy-10-(methoxycarbonyl)-8-methyl-8,16-diazapentacyclo[10.6.1.0^{1,9}.0^{2,7}.0^{16,19}]nonadeca-2(7),3,5,13-tetraen-16-ium + acetyl-CoA = (1R,9R,10S,11R,12R,19R)-11-(acetyloxy)-12-ethyl-10-hydroxy-5-methoxy-10-(methoxycarbonyl)-8-methyl-8,16-diazapentacyclo[10.6.1.0^{1,9}.0^{2,7}.0^{16,19}]nonadeca-2(7),3,5,13-tetraen-16-ium + CoA. Also known as: 17-O-deacetylvindoline-17-O-acetyltransferase activity, DAT activity, acetyl-CoA-17-O-deacetylvindoline 17-O-acetyltransferase activity, acetyl-CoA:17-O-deacetylvindoline 17-O-acetyltransferase activity, acetyl-CoA:deacetylvindoline 4-O-acetyltransferase activity, acetylcoenzyme A-deacetylvindoline 4-O-acetyltransferase activity, acetylcoenzyme A:deacetylvindoline 4-O-acetyltransferase activity, acetylcoenzyme A:deacetylvindoline O-acetyltransferase activity, deacetylvindoline O-acetyltransferase activity, deacetylvindoline acetyltransferase activity